{
  "gene": "UniProtKB:C9JLJ4",
  "term_id": "GO:0004843",
  "gene_name": "Ubiquitin carboxyl-terminal hydrolase 17-like protein 13",
  "gene_symbol": "USP17L13",
  "term_label": "cysteine-type deubiquitinase activity"
}